{
  "gene": "UniProtKB:Q8TCG5",
  "gene_name": "Carnitine O-palmitoyltransferase 1, brain isoform",
  "gene_symbol": "CPT1C",
  "term_id": "GO:0005789",
  "term_label": "endoplasmic reticulum membrane"
}